mesectoderm development [GO:0048383] (biological process) Definition: The process whose specific outcome is the progression of the mesectoderm over time, from its formation to the mature structure. In animal embryos, mesectoderm development processes give rise to both mesoderm and ectoderm tissues. Sources: GOC:jid Relationships: is a type of GO:0009888; is part of ectoderm development [GO:0007398]; is part of mesoderm development [GO:0007498]